succinylglutamate-semialdehyde dehydrogenase activity [GO:0043824] (molecular function) Also known as: succinyl glutamate-semialdehyde dehydrogenase activity, AruD, AstD, N-succinyl-L-glutamate 5-semialdehyde:NAD+ oxidoreductase activity, N-succinylglutamate 5-semialdehyde dehydrogenase activity, SGSD, succinylglutamic semialdehyde dehydrogenase activity Relationships: is a type of oxidoreductase activity, acting on the aldehyde or oxo group of donors, NAD or NADP as acceptor [GO:0016620] Definition: Catalysis of the reaction: N-succinyl-L-glutamate 5-semialdehyde + H2O + NAD+ = N-succinyl-L-glutamate + 2 H+ + NADH. Sources: EC:1.2.1.71, RHEA:10812